{
  "term_label": "centriole",
  "term_id": "GO:0005814",
  "gene_symbol": "CNTROB",
  "gene_name": "Centrobin",
  "gene": "UniProtKB:Q8N137"
}